{
  "term_id": "GO:0032456",
  "gene_name": "EH domain-containing protein 1",
  "term_label": "endocytic recycling",
  "gene_symbol": "EHD1",
  "gene": "UniProtKB:Q9H4M9"
}